{
  "term_id": "UNKNOWN:0003",
  "gene": "UniProtKB:Q9NVH1",
  "gene_name": "DnaJ homolog subfamily C member 11",
  "gene_symbol": "DNAJC11",
  "term_label": "Unknown cellular component"
}